{
  "term_id": "GO:0160224",
  "gene_name": "5-demethoxyubiquinone hydroxylase, mitochondrial",
  "gene": "UniProtKB:Q99807",
  "gene_symbol": "COQ7",
  "term_label": "3-demethoxyubiquinone 3-hydroxylase (NADH) activity"
}